{
  "term_label": "nucleus",
  "gene_name": "Zinc finger protein 586",
  "gene_symbol": "ZNF586",
  "term_id": "GO:0005634",
  "gene": "UniProtKB:Q9NXT0"
}